{
  "term_label": "phosphatidylinositol-4,5-bisphosphate binding",
  "gene_name": "APC membrane recruitment protein 3",
  "term_id": "GO:0005546",
  "gene_symbol": "AMER3",
  "gene": "UniProtKB:Q8N944"
}